{
  "term_id": "GO:0005886",
  "gene_name": "Disintegrin and metalloproteinase domain-containing protein 20",
  "gene": "UniProtKB:O43506",
  "gene_symbol": "ADAM20",
  "term_label": "plasma membrane"
}